{
  "gene_name": "Envoplakin",
  "term_id": "GO:0005882",
  "gene_symbol": "EVPL",
  "term_label": "intermediate filament",
  "gene": "UniProtKB:Q92817"
}